{
  "term_label": "RNA polymerase II cis-regulatory region sequence-specific DNA binding",
  "term_id": "GO:0000978",
  "gene_symbol": "BCL6B",
  "gene": "UniProtKB:Q8N143",
  "gene_name": "B-cell CLL_lymphoma 6 member B protein"
}